{
  "term_id": "GO:0004252",
  "gene_name": "Proprotein convertase subtilisin_kexin type 6",
  "gene_symbol": "PCSK6",
  "gene": "UniProtKB:P29122",
  "term_label": "serine-type endopeptidase activity"
}